{
  "term_id": "GO:0072659",
  "term_label": "protein localization to plasma membrane",
  "gene_name": "Ankyrin-1",
  "gene_symbol": "ANK1",
  "gene": "UniProtKB:P16157"
}